{
  "term_id": "GO:0005549",
  "gene": "UniProtKB:Q8NGG8",
  "term_label": "odorant binding",
  "gene_name": "Olfactory receptor 8B3",
  "gene_symbol": "OR8B3"
}